mammary gland bud morphogenesis [GO:0060648] (biological process) References: PMID:12558599 Sources: GOC:dph Definition: The process in which anatomical structures of the mammary gland buds are generated and organized. Mammary gland buds form by an outpocketing of the mammary placodes and grow to invade the mammary fat, when they form the mammary cord. Relationships: is_a morphogenesis of an epithelial bud [GO:0060572]; is part of mammary gland duct morphogenesis [GO:0060603]